{
  "term_id": "UNKNOWN:0002",
  "term_label": "Unknown biological process",
  "gene": "UniProtKB:A0A075B700",
  "gene_symbol": "TRAJ31",
  "gene_name": "T cell receptor alpha joining 31"
}